{
  "gene_name": "Nocturnin",
  "term_id": "GO:0000175",
  "gene": "UniProtKB:Q9UK39",
  "gene_symbol": "NOCT",
  "term_label": "3'-5'-RNA exonuclease activity"
}